{
  "gene": "UniProtKB:Q96C92",
  "term_id": "GO:0055037",
  "gene_name": "Endosome-associated-trafficking regulator 1",
  "gene_symbol": "ENTR1",
  "term_label": "recycling endosome"
}